{
  "gene_symbol": "FGF10",
  "gene_name": "Fibroblast growth factor 10",
  "gene": "UniProtKB:O15520",
  "term_id": "GO:0005737",
  "term_label": "cytoplasm"
}